titin-telethonin complex [GO:1990733] (cellular component) Note: An example of this are TTN and TCAP in human (UniProt symbols Q8WZ42 and O15273 respectively) in PMID:16407954 (inferred from direct assay). Also known as: Titin-Tcap complex Relationships: is a type of protein-containing complex [GO:0032991]; BFO_0000050 GO:0030018 Definition: A protein complex formed between the N-terminus of the giant sarcomeric filament protein titin and the Z-disk ligand, telethonin. The complex is part of the Z-disk of the skeletal and cardiac sarcomere. Telethonin binding to titin might be essential for the initial assembly, stabilization and functional integrity of the titin filament, and hence important for muscle contraction relaxation in mature myofibrils. References: PMID:16407954 Sources: GOC:ame